4-aminobutyrate transaminase complex [GO:0032144] (cellular component) Definition: A homodimeric protein complex that possesses 4-aminobutyrate transaminase activity. References: PMID:15528998 Sources: GOC:mah Also known as: ABAT complex, GABA transaminase complex, GABA-T complex Relationships: is a type of intracellular protein-containing complex [GO:0140535]; is a type of transferase complex [GO:1990234]